{
  "gene_name": "Phospholipase A and acyltransferase 3",
  "term_label": "phospholipase A2 activity",
  "gene_symbol": "PLAAT3",
  "term_id": "GO:0004623",
  "gene": "UniProtKB:P53816"
}